N-acyl-D-amino-acid deacylase activity [GO:0047420] (molecular function) Sources: EC:3.5.1.81, MetaCyc:3.5.1.81-RXN Also known as: D-aminoacylase activity, N-acyl-D-amino acid amidohydrolase activity Relationships: is a type of GO:0016811 Definition: Catalysis of the reaction: H2O + N-acyl-D-amino acid = D-amino acid + an acid.